sperm entry [GO:0035037] (biological process) Definition: An endocytosis process that results in penetration of the egg shell through the micropyle (a specialized anterior opening in the vitelline envelope) and entry of the entire sperm, including the surrounding plasma membrane and the sperm tail, into the egg cytoplasm. This step in fertilization is seen in Drosophila, where a plasma membrane fusion event between the sperm and the egg does not occur. References: PMID:9630751 Sources: GOC:bf Relationships: is a type of endocytosis [GO:0006897]; BFO_0000050 single fertilization [GO:0007338]